regulation of plant-type cell wall cellulose catabolic process [GO:2000939] (biological process) Subtypes: negative regulation of plant-type cell wall cellulose catabolic process [GO:2000940], positive regulation of plant-type cell wall cellulose catabolic process [GO:2000941] Also known as: regulation of plant-type cell wall polysaccharide breakdown Relationships: is a type of regulation of beta-glucan metabolic process [GO:0032950]; is a type of regulation of cell wall polysaccharide catabolic process [GO:2000966]; regulates plant-type cell wall cellulose catabolic process [GO:0044348] Sources: GOC:mengo_curators Definition: Any process that modulates the frequency, rate or extent of plant-type cell wall cellulose catabolic process.